venom-mediated inhibition of voltage-gated potassium channel activity [GO:0044562] (biological process) Relationships: is a type of venom-mediated perturbation of voltage-gated potassium channel activity [GO:0044559] Definition: A process in which an organism inhibits or disrupts the activity of a  voltage-gated potassium channel in another organism via the action of a venom. Sources: GOC:fj, GOC:jl Also known as: envenomation resulting in negative regulation of voltage-gated potassium channel activity in another organism, envenomation resulting in negative regulation of voltage-gated potassium channel activity in other organism